{
  "gene_symbol": "SPDYE7P",
  "gene_name": "Putative speedy protein E7",
  "term_label": "protein kinase binding",
  "gene": "UniProtKB:Q495Y7",
  "term_id": "GO:0019901"
}